{
  "gene_name": "Inositol polyphosphate-4-phosphatase type I A",
  "term_id": "GO:0005737",
  "gene": "UniProtKB:Q96PE3",
  "gene_symbol": "INPP4A",
  "term_label": "cytoplasm"
}